positive regulation of defecation rhythm [GO:2000748] (biological process) Definition: Any process that activates or increases the frequency, rate or extent of defecation rhythm. Relationships: is a type of positive regulation of defecation [GO:2000294]; is a type of regulation of defecation rhythm [GO:2000746]; positively regulates defecation rhythm [GO:0035882] Sources: GOC:kmv Also known as: positive regulation of DMP, positive regulation of defecation cycle, positive regulation of defecation motor program, positive regulation of defecation behavior